oligosaccharide transmembrane transporter activity [GO:0015157] (molecular function) Definition: Enables the transfer of oligosaccharide from one side of a membrane to the other. Sources: GOC:jl, GOC:mtg_transport, ISBN:0815340729 Also known as: endosomal oligosaccharide transporter Relationships: is a type of carbohydrate transmembrane transporter activity [GO:0015144]; BFO_0000050 oligosaccharide transport [GO:0015772] Subtypes: disaccharide transmembrane transporter activity [GO:0015154], raffinose transmembrane transporter activity [GO:0015158], ABC-type oligosaccharide transporter activity [GO:0015422], oligosaccharide transporting porin activity [GO:0015478]